{
  "gene_symbol": "OR4L1",
  "term_label": "Unknown cellular component",
  "term_id": "UNKNOWN:0003",
  "gene_name": "Olfactory receptor 4L1",
  "gene": "UniProtKB:Q8NH43"
}